galactolipid O-acyltransferase activity [GO:0047909] (molecular function) Definition: Catalysis of the reaction: 2 mono-beta-D-galactosyldiacylglycerol = acylmono-beta-D-galactosyl-diacylglycerol + mono-beta-D-galactosylacylglycerol. Relationships: is a type of GO:0008374 Also known as: galactolipid:galactolipid acyltransferase activity, mono-beta-D-galactosyldiacylglycerol:mono-beta-D-galactosyldiacylglycerol acyltransferase activity Sources: EC:2.3.1.134, MetaCyc:GALACTOLIPID-O-ACYLTRANSFERASE-RXN